{
  "term_id": "UNKNOWN:0003",
  "term_label": "Unknown cellular component",
  "gene_symbol": "NDUFV1-DT",
  "gene_name": "Uncharacterized protein NDUFV1-DT",
  "gene": "UniProtKB:Q8NBR9"
}